{
  "term_id": "UNKNOWN:0003",
  "gene_name": "Unconventional prefoldin RPB5 interactor 1",
  "gene": "UniProtKB:O94763",
  "gene_symbol": "URI1",
  "term_label": "Unknown cellular component"
}